{
  "gene_symbol": "INS-IGF2",
  "term_id": "GO:0005179",
  "term_label": "hormone activity",
  "gene_name": "Insulin, isoform 2",
  "gene": "UniProtKB:F8WCM5"
}